{
  "gene_name": "AT-rich interactive domain-containing protein 3A",
  "term_id": "GO:0005634",
  "gene_symbol": "ARID3A",
  "gene": "UniProtKB:Q99856",
  "term_label": "nucleus"
}